{
  "gene": "UniProtKB:Q9H7P9",
  "gene_symbol": "PLEKHG2",
  "gene_name": "Pleckstrin homology domain-containing family G member 2",
  "term_id": "GO:0030833",
  "term_label": "regulation of actin filament polymerization"
}